{
  "gene_name": "Importin-9",
  "gene_symbol": "IPO9",
  "term_label": "protein import into nucleus",
  "gene": "UniProtKB:Q96P70",
  "term_id": "GO:0006606"
}